{
  "gene": "UniProtKB:Q8IW40",
  "gene_name": "Coiled-coil domain-containing protein 103",
  "gene_symbol": "CCDC103",
  "term_id": "UNKNOWN:0001",
  "term_label": "Unknown molecular function"
}